{
  "term_label": "apical plasma membrane",
  "gene_name": "Probable small intestine urate exporter",
  "gene_symbol": "SLC17A4",
  "gene": "UniProtKB:Q9Y2C5",
  "term_id": "GO:0016324"
}